{
  "gene": "UniProtKB:Q6P9H4",
  "gene_symbol": "CNKSR3",
  "gene_name": "Connector enhancer of kinase suppressor of ras 3",
  "term_label": "Unknown cellular component",
  "term_id": "UNKNOWN:0003"
}